{
  "term_label": "transmembrane transporter complex",
  "gene_symbol": "HTR3A",
  "term_id": "GO:1902495",
  "gene": "UniProtKB:P46098",
  "gene_name": "5-hydroxytryptamine receptor 3A"
}